{
  "term_label": "dimethylglycine dehydrogenase activity",
  "gene_symbol": "DMGDH",
  "gene": "UniProtKB:Q9UI17",
  "term_id": "GO:0047865",
  "gene_name": "Dimethylglycine dehydrogenase, mitochondrial"
}